{
  "gene_symbol": "RGS7BP",
  "gene_name": "Regulator of G-protein signaling 7-binding protein",
  "term_label": "nucleus",
  "gene": "UniProtKB:Q6MZT1",
  "term_id": "GO:0005634"
}